{
  "term_id": "GO:0000139",
  "gene": "UniProtKB:O96024",
  "gene_symbol": "B3GALT4",
  "gene_name": "Beta-1,3-galactosyltransferase 4",
  "term_label": "Golgi membrane"
}